{
  "term_id": "GO:0051123",
  "gene": "UniProtKB:Q01658",
  "gene_name": "Protein Dr1",
  "term_label": "RNA polymerase II preinitiation complex assembly",
  "gene_symbol": "DR1"
}